{
  "term_label": "ATPase activator activity",
  "gene_name": "Activator of 90 kDa heat shock protein ATPase homolog 1",
  "gene": "UniProtKB:O95433",
  "gene_symbol": "AHSA1",
  "term_id": "GO:0001671"
}